{
  "gene": "UniProtKB:O75771",
  "gene_symbol": "RAD51D",
  "term_id": "GO:0005815",
  "term_label": "microtubule organizing center",
  "gene_name": "DNA repair protein RAD51 homolog 4"
}